{
  "term_id": "GO:0047757",
  "gene_name": "Dermatan-sulfate epimerase",
  "gene": "UniProtKB:Q9UL01",
  "gene_symbol": "DSE",
  "term_label": "chondroitin-glucuronate 5-epimerase activity"
}